{
  "term_id": "GO:0005634",
  "gene_name": "MAP kinase-interacting serine_threonine-protein kinase 1",
  "gene_symbol": "MKNK1",
  "term_label": "nucleus",
  "gene": "UniProtKB:Q9BUB5"
}